{
  "term_label": "Unknown molecular function",
  "gene_symbol": "ATP5MC1",
  "gene_name": "ATP synthase F(0) complex subunit C1, mitochondrial",
  "gene": "UniProtKB:P05496",
  "term_id": "UNKNOWN:0001"
}